{
  "gene_symbol": "TCEAL8",
  "term_id": "UNKNOWN:0003",
  "gene_name": "Transcription elongation factor A protein-like 8",
  "gene": "UniProtKB:Q8IYN2",
  "term_label": "Unknown cellular component"
}